{
  "term_id": "GO:0032266",
  "gene": "UniProtKB:Q9Y484",
  "gene_symbol": "WDR45",
  "gene_name": "WD repeat domain phosphoinositide-interacting protein 4",
  "term_label": "phosphatidylinositol-3-phosphate binding"
}